{
  "term_id": "UNKNOWN:0003",
  "term_label": "Unknown cellular component",
  "gene_name": "Protein phosphatase 1 regulatory subunit 36",
  "gene_symbol": "PPP1R36",
  "gene": "UniProtKB:Q96LQ0"
}